{
  "gene_name": "Protein phosphatase inhibitor 2",
  "gene_symbol": "PPP1R2",
  "gene": "UniProtKB:P41236",
  "term_label": "protein phosphatase inhibitor activity",
  "term_id": "GO:0004864"
}